{
  "term_label": "6-phosphofructokinase complex",
  "term_id": "GO:0005945",
  "gene_symbol": "PFKP",
  "gene": "UniProtKB:Q01813",
  "gene_name": "ATP-dependent 6-phosphofructokinase, platelet type"
}